{
  "term_id": "UNKNOWN:0003",
  "gene_symbol": "NTN1",
  "gene": "UniProtKB:O95631",
  "term_label": "Unknown cellular component",
  "gene_name": "Netrin-1"
}